protein-RNA complex assembly [GO:0022618] (biological process) Also known as: RNA-protein complex assembly, RNP complex assembly, ribonucleoprotein complex assembly Subtypes: ribosomal large subunit assembly [GO:0000027], ribosomal small subunit assembly [GO:0000028], spliceosomal complex assembly [GO:0000245], mRNA branch site recognition [GO:0000348], generation of catalytic spliceosome for first transesterification step [GO:0000349], generation of catalytic spliceosome for second transesterification step [GO:0000350], GO:0000352, formation of quadruple SL/U4/U5/U6 snRNP [GO:0000353], cis assembly of pre-catalytic spliceosome [GO:0000354], GO:0000387, spliceosome conformational change to release U4 (or U4atac) and U1 (or U11) [GO:0000388], GO:0000393, small nucleolar ribonucleoprotein complex assembly [GO:0000491], formation of translation initiation ternary complex [GO:0001677], GO:0001731, GO:0001732, GO:0006376, small-subunit processome assembly [GO:0034462], 90S preribosome assembly [GO:0034463], RISC complex assembly [GO:0070922], assembly of large subunit precursor of preribosome [GO:1902626], RITS complex assembly [GO:1904802], telomerase holoenzyme complex assembly [GO:1905323], cytoplasmic U snRNP body assembly [GO:1990194] Relationships: is a type of protein-containing complex assembly [GO:0065003]; is a type of protein-RNA complex organization [GO:0071826]; BFO_0000050 ribonucleoprotein complex biogenesis [GO:0022613] Sources: GOC:jl Definition: The aggregation, arrangement and bonding together of proteins and RNA molecules to form a ribonucleoprotein complex.